{
  "gene_symbol": "RC3H1",
  "term_id": "GO:0010494",
  "term_label": "cytoplasmic stress granule",
  "gene_name": "Roquin-1",
  "gene": "UniProtKB:Q5TC82"
}